box C/D methylation guide scaRNP complex [GO:0170051] (cellular component) References: PMID:27775477 Definition: A ribonucleoprotein complex containing a small CB-specific RNA (scaRNA), with a short sequence motif (GU/UG wobble stem) for CB localization that is capable of methylation of target RNAs. Relationships: is a type of box C/D RNP complex [GO:0170049]